{
  "gene_symbol": "WDR24",
  "gene_name": "GATOR complex protein WDR24",
  "term_id": "GO:0061700",
  "gene": "UniProtKB:Q96S15",
  "term_label": "GATOR2 complex"
}